Swi5-Sfr1 complex [GO:0032798] (cellular component) Also known as: Swi5 complex, Sae3-Mei5 complex References: PMID:15620352, PMID:16921379 Note: Note that this term refers to Schizosaccharomyces pombe Swi5, which should not be confused with the unrelated Saccharomyces Swi5p. Relationships: is a type of DNA recombinase mediator complex [GO:0033061]; is a type of nuclear protein-containing complex [GO:0140513]; is part of GO:0000228; is part of chromatin [GO:0000785] Definition: A conserved DNA recombinase mediator complex that contains two Swi5 monomers and one Sfr1 monomer in Schizosaccharomyces, or orthologs thereof (e.g. Sae3p and Mei5p in Saccharomyces).